{
  "gene": "UniProtKB:O96019",
  "gene_name": "Actin-like protein 6A",
  "term_label": "regulation of transcription by RNA polymerase II",
  "gene_symbol": "ACTL6A",
  "term_id": "GO:0006357"
}